{
  "gene_name": "Adhesion G protein-coupled receptor F4",
  "term_id": "UNKNOWN:0003",
  "gene": "UniProtKB:Q8IZF3",
  "term_label": "Unknown cellular component",
  "gene_symbol": "ADGRF4"
}